{
  "term_id": "GO:0097020",
  "gene": "UniProtKB:Q6UWH6",
  "term_label": "COPII receptor activity",
  "gene_name": "Protein TEX261",
  "gene_symbol": "TEX261"
}